{
  "term_label": "enzyme-substrate adaptor activity",
  "term_id": "GO:0140767",
  "gene_symbol": "CDC16",
  "gene_name": "Cell division cycle protein 16 homolog",
  "gene": "UniProtKB:Q13042"
}